negative regulation of cytoplasmic translational elongation [GO:1900248] (biological process) Definition: Any process that stops, prevents or reduces the frequency, rate or extent of cytoplasmic translational elongation. Relationships: is a type of GO:0045900; is a type of regulation of cytoplasmic translational elongation [GO:1900247]; is a type of negative regulation of cytoplasmic translation [GO:2000766]; negatively regulates cytoplasmic translational elongation [GO:0002182] Subtypes: negative regulation of cytoplasmic translational elongation through polyproline stretches [GO:1903271] Also known as: down regulation of cytoplasmic translational elongation, down-regulation of cytoplasmic translational elongation, downregulation of cytoplasmic translational elongation, inhibition of cytoplasmic translational elongation Sources: GOC:TermGenie